{
  "gene_symbol": "PNCK",
  "term_label": "calcium/calmodulin-dependent protein kinase activity",
  "term_id": "GO:0004683",
  "gene": "UniProtKB:Q6P2M8",
  "gene_name": "Calcium_calmodulin-dependent protein kinase type 1B"
}